{
  "gene": "UniProtKB:A4D1Z8",
  "term_label": "Unknown cellular component",
  "gene_symbol": "GRIFIN",
  "term_id": "UNKNOWN:0003",
  "gene_name": "Grifin"
}